{
  "gene_name": "C-C chemokine receptor type 1",
  "term_label": "inflammatory response",
  "gene": "UniProtKB:P32246",
  "term_id": "GO:0006954",
  "gene_symbol": "CCR1"
}